{
  "term_id": "GO:0005737",
  "gene_symbol": "EGLN2",
  "gene_name": "Prolyl hydroxylase EGLN2",
  "gene": "UniProtKB:Q96KS0",
  "term_label": "cytoplasm"
}